{
  "gene_name": "Putative adhesion G protein-coupled receptor E4P",
  "term_label": "G protein-coupled receptor signaling pathway",
  "gene_symbol": "ADGRE4P",
  "gene": "UniProtKB:Q86SQ3",
  "term_id": "GO:0007186"
}